{
  "term_label": "Unknown biological process",
  "gene_name": "Zinc finger protein 385D",
  "term_id": "UNKNOWN:0002",
  "gene": "UniProtKB:Q9H6B1",
  "gene_symbol": "ZNF385D"
}